non-canonical Wnt signaling pathway [GO:0035567] (biological process) Note: This term should only be used when Wnt receptor signaling occurs via a beta-catenin-independent route but the downstream effectors are unknown. If the downstream effectors are known, consider instead annotating to one of the children, or requesting a new term. References: PMID:37804416 Relationships: is_a GO:0016055 Also known as: beta-catenin-independent Wnt receptor signaling pathway, non-canonical Wnt receptor signaling pathway, non-canonical Wnt receptor signalling pathway, non-canonical Wnt-activated signaling pathway Subtypes: Wnt signaling pathway, calcium modulating pathway [GO:0007223], GO:0060069, GO:0060071, non-canonical Wnt signaling pathway involved in heart development [GO:0061341], Frizzled Nuclear Import pathway [GO:0140709] Regulation: regulated by regulation of non-canonical Wnt signaling pathway [GO:2000050]; negatively regulated by negative regulation of non-canonical Wnt signaling pathway [GO:2000051]; positively regulated by GO:2000052 Definition: A type of Wnt signaling pathway in which Wnt binding to its receptor on the surface of a target cell results in the by propagation of the molecular signals via effectors other than beta-catenin.